{
  "gene_symbol": "SP5",
  "term_id": "GO:0000978",
  "gene": "UniProtKB:Q6BEB4",
  "gene_name": "Transcription factor Sp5",
  "term_label": "RNA polymerase II cis-regulatory region sequence-specific DNA binding"
}